{
  "gene_name": "Deoxyribonuclease-2-beta",
  "gene_symbol": "DNASE2B",
  "gene": "UniProtKB:Q8WZ79",
  "term_label": "Unknown cellular component",
  "term_id": "UNKNOWN:0003"
}